negative regulation of conjugation with cellular fusion [GO:0031138] (biological process) Also known as: down regulation of conjugation with cellular fusion, down-regulation of conjugation with cellular fusion, downregulation of conjugation with cellular fusion, inhibition of conjugation with cellular fusion Relationships: is a type of regulation of conjugation with cellular fusion [GO:0031137]; is a type of negative regulation of reproductive process [GO:2000242]; negatively regulates conjugation with cellular fusion [GO:0000747] Sources: GOC:mah Subtypes: negative regulation of induction of conjugation with cellular fusion [GO:0010515], negative regulation of conjugation with zygote [GO:0140538] Definition: Any process that decreases the rate or frequency of conjugation with cellular fusion.